secondary cell wall biogenesis involved in seed trichome differentiation [GO:0090379] (biological process) Also known as: secondary cell wall biosynthesis involved in seed trichome differentiation, seed trichome secondary wall biosynthesis Sources: GOC:tb Relationships: is a type of plant-type secondary cell wall biogenesis [GO:0009834]; is part of GO:0090376 Note: The processes involved in the massive amount of secondary wall cellulose synthesis in seed trichomes continue to 30 DPA in Gossypium spp. Definition: A cellular process that results in the biosynthesis of constituent macromolecules, assembly, and arrangement of constituent parts of inextensible cellulose- and pectin-containing cell walls that are formed between the plasma membrane and primary cell wall of seed trichomes after cell expansion is complete.